{
  "term_id": "GO:0005615",
  "gene_name": "Proto-oncogene Wnt-3",
  "gene_symbol": "WNT3",
  "term_label": "extracellular space",
  "gene": "UniProtKB:P56703"
}